{
  "gene": "UniProtKB:Q96MV1",
  "term_label": "endoplasmic reticulum",
  "term_id": "GO:0005783",
  "gene_symbol": "TLCD4",
  "gene_name": "TLC domain-containing protein 4"
}